{
  "term_id": "GO:0005743",
  "gene_symbol": "SFXN2",
  "gene": "UniProtKB:Q96NB2",
  "gene_name": "Sideroflexin-2",
  "term_label": "mitochondrial inner membrane"
}